{
  "gene": "UniProtKB:Q8N6W0",
  "gene_name": "CUGBP Elav-like family member 5",
  "term_label": "mRNA binding",
  "term_id": "GO:0003729",
  "gene_symbol": "CELF5"
}